{
  "term_id": "GO:0004984",
  "gene_name": "Olfactory receptor 2T6",
  "term_label": "olfactory receptor activity",
  "gene_symbol": "OR2T6",
  "gene": "UniProtKB:Q8NHC8"
}